{
  "term_id": "GO:0005886",
  "gene_name": "Patched domain-containing protein 1",
  "gene": "UniProtKB:Q96NR3",
  "gene_symbol": "PTCHD1",
  "term_label": "plasma membrane"
}